phosphoserine residue binding [GO:0050815] (molecular function) Relationships: is_a protein phosphorylated amino acid binding [GO:0045309] Also known as: phosphoserine binding Subtypes: RNA polymerase II C-terminal domain phosphoserine binding [GO:1990269] Sources: GOC:ai Definition: Binding to a phosphorylated serine residue within a protein.